{
  "term_id": "GO:0005814",
  "gene_name": "Centrosome-associated protein CEP250",
  "gene": "UniProtKB:Q9BV73",
  "term_label": "centriole",
  "gene_symbol": "CEP250"
}